{
  "gene": "UniProtKB:P11912",
  "gene_symbol": "CD79A",
  "term_id": "GO:0019815",
  "term_label": "B cell receptor complex",
  "gene_name": "B-cell antigen receptor complex-associated protein alpha chain"
}